{
  "gene_symbol": "SOAT2",
  "gene_name": "Sterol O-acyltransferase 2",
  "gene": "UniProtKB:O75908",
  "term_label": "cholesterol efflux",
  "term_id": "GO:0033344"
}